chitosan layer of spore wall [GO:0005631] (cellular component) Definition: The second outermost layer of the spore wall, as described in Saccharomyces. Sources: ISBN:0879693568 Relationships: is a type of cellular anatomical structure [GO:0110165]; is part of ascospore wall [GO:0005619]